{
  "term_id": "GO:0005634",
  "term_label": "nucleus",
  "gene_name": "Protein ripply1",
  "gene_symbol": "RIPPLY1",
  "gene": "UniProtKB:Q0D2K3"
}